{
  "term_id": "GO:0008013",
  "term_label": "beta-catenin binding",
  "gene": "UniProtKB:P55287",
  "gene_name": "Cadherin-11",
  "gene_symbol": "CDH11"
}